nitric oxide production involved in inflammatory response [GO:0002537] (biological process) Sources: GOC:add, ISBN:0781735149 Also known as: nitric oxide production involved in acute inflammatory response, production of nitric oxide involved in acute inflammatory response, production of nitric oxide involved in inflammatory response Definition: The synthesis or release of nitric oxide following a stimulus as part of an inflammatory response, resulting in an increase in its intracellular or extracellular levels. Relationships: is a type of production of molecular mediator involved in inflammatory response [GO:0002532]